{
  "gene_symbol": "AMOT",
  "term_label": "cytoplasmic vesicle",
  "gene_name": "Angiomotin",
  "gene": "UniProtKB:Q4VCS5",
  "term_id": "GO:0031410"
}